{
  "term_label": "Unknown molecular function",
  "gene_name": "Coiled-coil domain-containing protein 97",
  "gene_symbol": "CCDC97",
  "gene": "UniProtKB:Q96F63",
  "term_id": "UNKNOWN:0001"
}